{
  "gene_name": "DNA excision repair protein ERCC-6-like 2",
  "term_label": "interstrand cross-link repair",
  "term_id": "GO:0036297",
  "gene": "UniProtKB:Q5T890",
  "gene_symbol": "ERCC6L2"
}